{
  "gene": "UniProtKB:Q6ZT77",
  "gene_name": "Putative zinc finger protein 826",
  "gene_symbol": "ZNF826P",
  "term_label": "Unknown cellular component",
  "term_id": "UNKNOWN:0003"
}